negative regulation melanotic encapsulation of foreign target [GO:0140540] (biological process) Relationships: is a type of GO:0002698; is_a negative regulation of melanization defense response [GO:0035009]; is a type of regulation of melanotic encapsulation of foreign target [GO:0140539]; negatively regulates melanotic encapsulation of foreign target [GO:0035011] References: PMID:15749104, PMID:18457993 Definition: Any process that stops, prevents or reduces the frequency, rate or extent of melanotic encapsulation of foreign target.